{
  "gene_symbol": "FITM1",
  "gene": "UniProtKB:A5D6W6",
  "term_id": "GO:0008654",
  "term_label": "phospholipid biosynthetic process",
  "gene_name": "Fat storage-inducing transmembrane protein 1"
}